cell projection [GO:0042995] (cellular component) References: PMID:16318917 Sources: GOC:jl Also known as: cell process, cellular process, cellular projection Subtypes: bacterial-type flagellum [GO:0009288], pilus [GO:0009289], haustorium [GO:0085035], plant cell papilla [GO:0090395], archaeal-type flagellum [GO:0097589], GO:0120025 Relationships: is a type of cellular anatomical structure [GO:0110165] Definition: A prolongation or process extending from a cell, e.g. a flagellum or axon.